{
  "gene_name": "PTEN upstream open reading frame MP31",
  "term_id": "UNKNOWN:0003",
  "gene": "UniProtKB:C0HLV8",
  "term_label": "Unknown cellular component",
  "gene_symbol": "C0HLV8"
}